{
  "gene": "UniProtKB:Q14980",
  "gene_symbol": "NUMA1",
  "term_id": "GO:0000132",
  "gene_name": "Nuclear mitotic apparatus protein 1",
  "term_label": "establishment of mitotic spindle orientation"
}